{
  "gene_name": "BTB_POZ domain-containing protein 18",
  "gene_symbol": "BTBD18",
  "gene": "UniProtKB:B2RXH4",
  "term_label": "Unknown molecular function",
  "term_id": "UNKNOWN:0001"
}